fruit septum development [GO:0080127] (BP) Definition: The process whose specific outcome is the progression of the fruit septum over time, from its formation to the mature structure. The fruit septum is a thin partition or membrane that divides a cavity or a mass of tissue in the fruit. Sources: GOC:dhl, PO:0005008 Relationships: is a type of developmental process involved in reproduction [GO:0003006]; is a type of post-embryonic development [GO:0009791]; is a type of plant septum development [GO:1905328]; is part of fruit development [GO:0010154]